{
  "term_id": "GO:0042276",
  "gene_symbol": "POLH",
  "term_label": "error-prone translesion synthesis",
  "gene_name": "DNA polymerase eta",
  "gene": "UniProtKB:Q9Y253"
}